signaling receptor regulator activity [GO:0030545] (molecular function) Sources: GOC:ceb Subtypes: GO:0030546, signaling receptor inhibitor activity [GO:0030547], neurotransmitter receptor regulator activity [GO:0099602] Definition: Binds to and modulates the activity of a receptor. Relationships: is a type of molecular function regulator activity [GO:0098772]; regulates signaling receptor activity [GO:0038023] Also known as: receptor regulator activity